{
  "gene_symbol": "ZNF491",
  "gene_name": "Zinc finger protein 491",
  "gene": "UniProtKB:Q8N8L2",
  "term_label": "RNA polymerase II transcription regulatory region sequence-specific DNA binding",
  "term_id": "GO:0000977"
}